Atg1/ULK1 kinase complex assembly [GO:1904745] (biological process) Relationships: is a type of protein-containing complex assembly [GO:0065003] Regulation: regulated by GO:1905864; negatively regulated by negative regulation of Atg1/ULK1 kinase complex assembly [GO:1905865]; positively regulated by positive regulation of Atg1/ULK1 kinase complex assembly [GO:1905866] References: PMID:25139988 Sources: GOC:TermGenie, GOC:dph, GO_REF:0000079 Definition: The aggregation, arrangement and bonding together of a set of components to form an Atg1/UKL1 kinase complex. Also known as: ATG1 kinase complex assembly, ATG1 kinase complex formation, ATG1-ATG13 complex assembly, ATG1-ATG13 complex formation, ATG1/ULK1 kinase complex formation, ATG1/ULK1 signaling complex assembly, ATG1/ULK1 signaling complex formation, Atg1p signalling complex assembly, Atg1p signalling complex formation, ULK1 signaling complex assembly, ULK1 signaling complex formation, ULK1-ATG13-FIP200 complex assembly, ULK1-ATG13-FIP200 complex formation, ULK1-ATG13-RB1CC1 complex assembly, ULK1-ATG13-RB1CC1 complex formation